{
  "gene_name": "Zinc finger protein 19",
  "term_label": "DNA-binding transcription factor activity, RNA polymerase II-specific",
  "gene": "UniProtKB:P17023",
  "gene_symbol": "ZNF19",
  "term_id": "GO:0000981"
}